{
  "gene_name": "Chromodomain-helicase-DNA-binding protein 7",
  "gene_symbol": "CHD7",
  "gene": "UniProtKB:Q9P2D1",
  "term_label": "DNA binding",
  "term_id": "GO:0003677"
}